{
  "gene_name": "C-C motif chemokine 24",
  "gene_symbol": "CCL24",
  "term_label": "chemokine-mediated signaling pathway",
  "gene": "UniProtKB:O00175",
  "term_id": "GO:0070098"
}